tRNA thio-modification [GO:0034227] (biological process) Subtypes: tRNA wobble position uridine thiolation [GO:0002143], tRNA 4-thiouridine biosynthesis [GO:0002937], mitochondrial tRNA thio-modification [GO:0070903] Definition: The addition a sulfur atom to a nucleotide in a tRNA molecule. References: PMID:12549933, PMID:14722066 Sources: GOC:mcc Also known as: tRNA thiolation Relationships: is a type of tRNA modification [GO:0006400]